{
  "gene": "UniProtKB:A6NMU1",
  "gene_name": "Olfactory receptor 52A4",
  "term_id": "GO:0005886",
  "term_label": "plasma membrane",
  "gene_symbol": "OR52A4P"
}